{
  "gene_name": "Nuclear factor interleukin-3-regulated protein",
  "term_id": "UNKNOWN:0001",
  "gene": "UniProtKB:Q16649",
  "term_label": "Unknown molecular function",
  "gene_symbol": "NFIL3"
}